{
  "gene_symbol": "SEL1L",
  "gene": "UniProtKB:Q9UBV2",
  "term_id": "GO:0005789",
  "gene_name": "Protein sel-1 homolog 1",
  "term_label": "endoplasmic reticulum membrane"
}